cytokine activity [GO:0005125] (molecular function) Definition: The activity of a soluble extracellular gene product that interacts with a receptor to effect a change in the activity of the receptor to control the survival, growth, differentiation and effector function of tissues and cells. References: PMID:11530802 Sources: ISBN:0198599471 Also known as: phytocytokine activity, autocrine activity, paracrine activity Relationships: is a type of receptor ligand activity [GO:0048018] Subtypes: GO:0008009 Regulation: regulated by regulation of cytokine activity [GO:0060300]; negatively regulated by negative regulation of cytokine activity [GO:0060302]